voltage-gated potassium channel activity involved in SA node cell action potential depolarization [GO:0086041] (molecular function) Sources: GOC:BHF, GOC:mtg_cardiac_conduct_nov11 Also known as: voltage-gated potassium channel activity involved in SAN cell action potential depolarization, voltage-gated potassium channel activity involved in sinoatrial node cell action potential depolarization, voltage-gated potassium channel activity involved in sinus node cell action potential depolarization Definition: Enables the transmembrane transfer of a potassium ion by a voltage-gated channel through the plasma membrane of an SA node cardiac muscle cell contributing to the depolarization phase of an action potential. A voltage-gated channel is a channel whose open state is dependent on the voltage across the membrane in which it is embedded. Relationships: is a type of voltage-gated potassium channel activity [GO:0005249]; is part of membrane depolarization during SA node cell action potential [GO:0086046]